{
  "gene_name": "GPI ethanolamine phosphate transferase 3",
  "term_id": "GO:0006506",
  "gene_symbol": "PIGO",
  "term_label": "GPI anchor biosynthetic process",
  "gene": "UniProtKB:Q8TEQ8"
}